positive regulation of single-species biofilm formation in or on host organism [GO:1900230] (biological process) Definition: Any process that activates or increases the frequency, rate or extent of single-species biofilm formation in or on host organism. Sources: GOC:TermGenie, GOC:di Relationships: is a type of positive regulation of single-species biofilm formation [GO:1900192]; is a type of regulation of single-species biofilm formation in or on host organism [GO:1900228]; positively regulates single-species biofilm formation in or on host organism [GO:0044407] Also known as: up regulation of single-species biofilm formation in or on host organism, up-regulation of single-species biofilm formation in or on host organism, upregulation of single-species biofilm formation in or on host organism, activation of single-species biofilm formation in or on host organism